{
  "gene": "UniProtKB:Q13084",
  "gene_symbol": "MRPL28",
  "term_id": "UNKNOWN:0002",
  "term_label": "Unknown biological process",
  "gene_name": "Large ribosomal subunit protein bL28m"
}